{
  "gene_symbol": "SPHKAP",
  "term_id": "GO:0005739",
  "gene": "UniProtKB:Q2M3C7",
  "term_label": "mitochondrion",
  "gene_name": "A-kinase anchor protein SPHKAP"
}